{
  "gene": "UniProtKB:P18509",
  "term_id": "GO:0043204",
  "gene_name": "Pituitary adenylate cyclase-activating polypeptide",
  "term_label": "perikaryon",
  "gene_symbol": "ADCYAP1"
}